{
  "gene": "UniProtKB:Q9Y2Y1",
  "term_id": "UNKNOWN:0001",
  "gene_name": "DNA-directed RNA polymerase III subunit RPC10",
  "term_label": "Unknown molecular function",
  "gene_symbol": "POLR3K"
}